{
  "term_id": "GO:0031123",
  "gene_name": "Poly(A) RNA polymerase GLD2",
  "term_label": "RNA 3'-end processing",
  "gene_symbol": "TENT2",
  "gene": "UniProtKB:Q6PIY7"
}